{
  "gene": "UniProtKB:Q9UQB3",
  "gene_symbol": "CTNND2",
  "term_label": "cadherin binding",
  "term_id": "GO:0045296",
  "gene_name": "Catenin delta-2"
}